{
  "term_label": "cytoplasm",
  "gene_name": "Metastasis-associated in colon cancer protein 1",
  "gene_symbol": "MACC1",
  "term_id": "GO:0005737",
  "gene": "UniProtKB:Q6ZN28"
}